{
  "term_id": "GO:0014704",
  "gene_name": "Plakophilin-2",
  "gene_symbol": "PKP2",
  "gene": "UniProtKB:Q99959",
  "term_label": "intercalated disc"
}